{
  "gene": "UniProtKB:P0C7P3",
  "term_id": "GO:0016075",
  "gene_name": "Protein SLFN14",
  "gene_symbol": "SLFN14",
  "term_label": "rRNA catabolic process"
}